cell wall modification [GO:0042545] (biological process) Sources: GOC:jl Subtypes: plant-type cell wall modification [GO:0009827], cell wall modification involved in multidimensional cell growth [GO:0042547], cell wall thickening [GO:0052386] Definition: The series of events leading to chemical and structural alterations of an existing cell wall that can result in loosening, increased extensibility or disassembly. Relationships: is a type of cell wall organization [GO:0071555]